{
  "gene": "UniProtKB:P14923",
  "gene_symbol": "JUP",
  "term_label": "nucleus",
  "gene_name": "Junction plakoglobin",
  "term_id": "GO:0005634"
}